{
  "gene_symbol": "IFT46",
  "gene_name": "Intraflagellar transport protein 46 homolog",
  "gene": "UniProtKB:Q9NQC8",
  "term_id": "UNKNOWN:0001",
  "term_label": "Unknown molecular function"
}